{
  "term_id": "GO:0030150",
  "gene": "UniProtKB:O14925",
  "term_label": "protein import into mitochondrial matrix",
  "gene_symbol": "TIMM23",
  "gene_name": "Mitochondrial import inner membrane translocase subunit Tim23"
}